{
  "gene_symbol": "UCP1",
  "term_label": "oxidative phosphorylation uncoupler activity",
  "term_id": "GO:0017077",
  "gene": "UniProtKB:P25874",
  "gene_name": "Mitochondrial brown fat uncoupling protein 1"
}